{
  "gene_name": "Hemoglobin subunit mu",
  "gene_symbol": "HBM",
  "term_id": "GO:0005833",
  "term_label": "hemoglobin complex",
  "gene": "UniProtKB:Q6B0K9"
}